{
  "gene_symbol": "MAFG",
  "term_label": "RNA polymerase II cis-regulatory region sequence-specific DNA binding",
  "term_id": "GO:0000978",
  "gene_name": "Transcription factor MafG",
  "gene": "UniProtKB:O15525"
}